{
  "gene_name": "Fructose-bisphosphate aldolase A",
  "term_id": "GO:0030388",
  "gene_symbol": "ALDOA",
  "term_label": "fructose 1,6-bisphosphate metabolic process",
  "gene": "UniProtKB:P04075"
}